{
  "gene_symbol": "PFN4",
  "gene": "UniProtKB:Q8NHR9",
  "term_label": "cell cortex",
  "term_id": "GO:0005938",
  "gene_name": "Profilin-4"
}